{
  "term_label": "Rab-protein geranylgeranyltransferase complex",
  "term_id": "GO:0005968",
  "gene_name": "Rab proteins geranylgeranyltransferase component A 2",
  "gene": "UniProtKB:P26374",
  "gene_symbol": "CHML"
}